{
  "term_id": "GO:0030154",
  "term_label": "cell differentiation",
  "gene": "UniProtKB:Q12841",
  "gene_name": "Follistatin-related protein 1",
  "gene_symbol": "FSTL1"
}